{
  "term_id": "GO:0043235",
  "term_label": "receptor complex",
  "gene": "UniProtKB:P46531",
  "gene_name": "Neurogenic locus notch homolog protein 1",
  "gene_symbol": "NOTCH1"
}